{
  "term_id": "GO:2000134",
  "gene_name": "Cyclin-dependent kinase 2-associated protein 2",
  "term_label": "negative regulation of G1/S transition of mitotic cell cycle",
  "gene": "UniProtKB:O75956",
  "gene_symbol": "CDK2AP2"
}